{
  "gene": "UniProtKB:Q96HP4",
  "term_id": "UNKNOWN:0001",
  "gene_name": "Oxidoreductase NAD-binding domain-containing protein 1",
  "gene_symbol": "OXNAD1",
  "term_label": "Unknown molecular function"
}